{
  "term_label": "nucleus",
  "gene_symbol": "H3-3B",
  "gene_name": "Histone H3.3",
  "gene": "UniProtKB:P84243",
  "term_id": "GO:0005634"
}